regulation of hormone levels [GO:0010817] (biological process) Definition: Any process that modulates the levels of hormone within an organism or a tissue. A hormone is any substance formed in very small amounts in one specialized organ or group of cells and carried (sometimes in the bloodstream) to another organ or group of cells in the same organism, upon which it has a specific regulatory action. Sources: GOC:BHF, GOC:dph, GOC:tb Relationships: is a type of regulation of biological quality [GO:0065008] Subtypes: regulation of angiotensin levels in blood [GO:0002002], GO:0009914, GO:0032350, hormone metabolic process [GO:0042445], regulation of hormone secretion [GO:0046883], regulation of auxin polar transport [GO:2000012]